interleukin-28 receptor binding [GO:0032003] (molecular function) Relationships: is a type of cytokine receptor binding [GO:0005126] Sources: GOC:rph Also known as: IL-28, interleukin-28 receptor ligand Definition: Binding to an interleukin-28 receptor.